orthogonal dichotomous subdivision of terminal units involved in lung branching morphogenesis [GO:0060488] (biological process) Also known as: perpendicular dichotomous subdivision of terminal units involved in lung branching morphogenesis Relationships: is a type of dichotomous subdivision of terminal units involved in lung branching [GO:0060448] Definition: The process in which a lung bud bifurcates perpendicular to the plane of the previous bud. Sources: GOC:dph, GOC:mtg_lung